{
  "gene": "UniProtKB:Q9HCE6",
  "gene_name": "Rho guanine nucleotide exchange factor 10-like protein",
  "gene_symbol": "ARHGEF10L",
  "term_id": "GO:0005085",
  "term_label": "guanyl-nucleotide exchange factor activity"
}